{
  "gene_name": "NF-kappa-B-repressing factor",
  "term_label": "nucleolus",
  "term_id": "GO:0005730",
  "gene": "UniProtKB:O15226",
  "gene_symbol": "NKRF"
}